{
  "term_id": "GO:0006308",
  "gene": "UniProtKB:Q92874",
  "term_label": "DNA catabolic process",
  "gene_name": "Deoxyribonuclease-1-like 2",
  "gene_symbol": "DNASE1L2"
}